{
  "term_label": "DNA-binding transcription factor activity",
  "gene_symbol": "ZNF350",
  "term_id": "GO:0003700",
  "gene_name": "Zinc finger protein 350",
  "gene": "UniProtKB:Q9GZX5"
}